{
  "term_id": "UNKNOWN:0003",
  "gene_name": "Nuclear receptor-binding factor 2",
  "gene_symbol": "NRBF2",
  "gene": "UniProtKB:Q96F24",
  "term_label": "Unknown cellular component"
}